regulation of cellular component organization [GO:0051128] (biological process) Sources: GOC:ai Subtypes: regulation of transcription open complex formation at RNA polymerase II promoter [GO:0001177], GO:0001558, GO:0010549, regulation of very-low-density lipoprotein particle remodeling [GO:0010901], regulation of endocytosis [GO:0030100], regulation of cell projection organization [GO:0031344], regulation of organelle organization [GO:0033043], regulation of plasma lipoprotein oxidation [GO:0034444], regulation of protein-containing complex disassembly [GO:0043244], regulation of protein-containing complex assembly [GO:0043254], regulation of intermediate filament polymerization or depolymerization [GO:0045108], GO:0046605, GO:0050807, negative regulation of cellular component organization [GO:0051129], positive regulation of cellular component organization [GO:0051130], regulation of syncytium formation by plasma membrane fusion [GO:0060142], regulation of fungal-type cell wall organization [GO:0060237], regulation of phospholipid translocation [GO:0061091], regulation of erythrocyte enucleation [GO:0061930], regulation of linear element assembly [GO:0090006], regulation of inclusion body assembly [GO:0090083], regulation of chylomicron remodeling [GO:0090318], regulation of cell-substrate junction organization [GO:0150116], regulation of hyaluranon cable assembly [GO:1900104], GO:1901626, regulation of synaptic vesicle membrane organization [GO:1901632], GO:1901888, GO:1901891, regulation of capsule organization [GO:1901913], regulation of chromatin organization [GO:1902275], GO:1902903, regulation of ascospore-type prospore membrane formation [GO:1903023], GO:1903053, regulation of vitellogenesis [GO:1903186], GO:1903329, regulation of adherens junction organization [GO:1903391], GO:1903729, regulation of fusion of virus membrane with host plasma membrane [GO:1903913], regulation of tight junction disassembly [GO:1905073], regulation of membrane invagination [GO:1905153], regulation of presynaptic active zone assembly [GO:1905518], regulation of blood microparticle formation [GO:2000332] Relationships: is a type of GO:0050794; regulates GO:0016043 Also known as: regulation of cellular component organisation, regulation of cell organisation, regulation of cell organization, regulation of cellular component organization and biogenesis Definition: Any process that modulates the frequency, rate or extent of a process involved in the formation, arrangement of constituent parts, or disassembly of cell structures, including the plasma membrane and any external encapsulating structures such as the cell wall and cell envelope.